{
  "gene": "UniProtKB:P58335",
  "term_id": "UNKNOWN:0002",
  "term_label": "Unknown biological process",
  "gene_name": "Anthrax toxin receptor 2",
  "gene_symbol": "ANTXR2"
}